lactoyl-CoA dehydratase activity [GO:0018819] (molecular function) Also known as: acrylyl coenzyme A hydratase activity, lactoyl coenzyme A dehydratase activity, lactoyl-CoA hydro-lyase (acryloyl-CoA-forming), lactoyl-CoA hydro-lyase activity, lactyl CoA dehydratase activity, lactyl-coenzyme A dehydrase activity Definition: Catalysis of the reaction: (R)-lactoyl-CoA = acryloyl-CoA + H2O. Sources: RHEA:34691 Relationships: is a type of hydro-lyase activity [GO:0016836]